{
  "term_label": "collagen fibril organization",
  "gene_symbol": "LOXL1",
  "term_id": "GO:0030199",
  "gene": "UniProtKB:Q08397",
  "gene_name": "Lysyl oxidase homolog 1"
}